viral terminase, large subunit [GO:0098009] (cellular component) Note: This term should only be used when the large subunit consists of more than one polypeptide. References: PMID:18687036 Sources: GOC:bm, GOC:ch, GOC:jh2 Also known as: virus terminase, large subunit Relationships: is a type of catalytic complex [GO:1902494]; is part of viral terminase complex [GO:0043493] Definition: The part of the viral terminase complex that contains the translocase and endonuclease activities and allows the translocation of the phage DNA into the procapsid. The large subunit usually assembles as a heterooligomer with the small subunit.